{
  "gene_symbol": "ADH1A",
  "gene": "UniProtKB:P07327",
  "term_id": "GO:0005829",
  "term_label": "cytosol",
  "gene_name": "Alcohol dehydrogenase 1A"
}